{
  "term_id": "GO:0095500",
  "gene": "UniProtKB:O43653",
  "gene_symbol": "PSCA",
  "gene_name": "Prostate stem cell antigen",
  "term_label": "acetylcholine receptor signaling pathway"
}